negative regulation of bacterial-type flagellum-dependent cell motility [GO:1902201] (biological process) Sources: GOC:TermGenie, GOC:cilia, GOC:jl Definition: Any process that stops, prevents or reduces the frequency, rate or extent of bacterial-type flagellum-dependent cell motility. Relationships: is a type of GO:1902021; is a type of negative regulation of cell motility [GO:2000146]; negatively regulates GO:0071973 Also known as: down regulation of bacterial-type flagellar cell motility, down regulation of flagellin-based flagellar cell motility, down-regulation of bacterial-type flagellar cell motility, down-regulation of flagellin-based flagellar cell motility, downregulation of bacterial-type flagellar cell motility, downregulation of flagellin-based flagellar cell motility, inhibition of flagellin-based flagellar cell motility, negative regulation of flagellin-based flagellar cell motility, inhibition of bacterial-type flagellar cell motility, negative regulation of bacterial-type flagellar cell motility